intracellular sulfate ion homeostasis [GO:0030642] (biological process) Relationships: is a type of GO:0055063; is a type of intracellular chemical homeostasis [GO:0055082] Also known as: sulphate ion homeostasis, cellular sulfate ion homeostasis References: PMID:24193406 Sources: GOC:mah Definition: A homeostatic process involved in the maintenance of a steady state level of sulfate ions within a cell.